maintenance of protein location in cell cortex of cell tip [GO:0097248] (biological process) Relationships: is a type of GO:0032065 References: PMID:19646873 Sources: GOC:al Definition: A process in which a protein or protein complex is maintained in a specific location in the cell cortex of a cell tip, and is prevented from moving elsewhere. The cell cortex of a cell tip is the region directly beneath the plasma membrane at either end of the longest axis of a cylindrical or elongated cell.